cellular response to electrical stimulus [GO:0071257] (biological process) Definition: Any process that results in a change in state or activity of a cell (in terms of movement, secretion, enzyme production, gene expression, etc.) as a result of an electrical stimulus. Relationships: is a type of GO:0051602; is a type of cellular response to abiotic stimulus [GO:0071214] Also known as: cellular response to electricity Sources: GOC:mah